smoothened signaling pathway involved in ventral spinal cord patterning [GO:0021910] (biological process) Definition: The series of molecular signals generated as a consequence of activation of the transmembrane protein Smoothened that results in the spatial identity of regions along the dorsal-ventral axis of the spinal cord. Relationships: is a type of smoothened signaling pathway [GO:0007224]; is part of spinal cord dorsal/ventral patterning [GO:0021513] Regulation: negatively regulated by GO:0021914 References: PMID:11262869 Sources: GOC:cls, GOC:dgh, GOC:dph, GOC:jid, GOC:tb Subtypes: smoothened signaling pathway involved in ventral spinal cord interneuron specification [GO:0021775], GO:0021776 Also known as: hedgehog signaling pathway involved in ventral spinal cord patterning, hh signaling pathway involved in ventral spinal cord patterning, smoothened signalling pathway in ventral spinal cord patterning